P-type calcium transporter activity involved in regulation of postsynaptic cytosolic calcium ion concentration [GO:1905059] (molecular function) References: PMID:20678993 Sources: GOC:TermGenie, GO_REF:0000061 Also known as: ATP phosphohydrolase (Ca2+-transporting) involved in regulation of postsynaptic cytosolic calcium ion concentration, ATPase-coupled calcium ion transmembrane transporter activity involved in regulation of postsynaptic cytosolic calcium levels, Ca(2+)-transporting ATPase activity involved in regulation of postsynaptic cytosolic calcium ion concentration, Ca2+-pumping ATPase activity involved in regulation of postsynaptic cytosolic calcium ion concentration, Ca2+-transporting ATPase activity involved in regulation of postsynaptic cytosolic calcium ion concentration, calcium transporting ATPase activity involved in regulation of postsynaptic cytosolic calcium ion concentration, calcium-transporting ATPase activity involved in regulation of postsynaptic cytosolic calcium ion concentration, calcium-transporting ATPase activity involved in regulation of postsynaptic cytosolic calcium levels, calcium ABC transporter involved in regulation of postsynaptic cytosolic calcium ion concentration, calcium efflux ATPase involved in regulation of postsynaptic cytosolic calcium ion concentration, calcium-translocating P-type ATPase activity involved in regulation of postsynaptic cytosolic calcium ion concentration, plasma membrane Ca-ATPase involved in regulation of postsynaptic cytosolic calcium ion concentration, sarco(endo)plasmic reticulum Ca2+-ATPase involved in regulation of postsynaptic cytosolic calcium ion concentration, sarcoplasmic reticulum ATPase involved in regulation of postsynaptic cytosolic calcium ion concentration Relationships: is a type of P-type calcium transporter activity [GO:0005388]; is part of regulation of postsynaptic cytosolic calcium ion concentration [GO:0099566] Definition: A calcium-transporting P-type ATPase activity involved in regulation of postsynaptic cytosolic calcium ion concentration.